secretory granule localization [GO:0032252] (biological process) Sources: GOC:mah Also known as: secretory granule localisation, secretory granule clustering Definition: Any process in which a secretory granule is transported to, and/or maintained in, a specific location within the cell. Relationships: is a type of GO:0051648 Subtypes: dense core granule localization [GO:0032253]